{
  "gene_symbol": "APBA2",
  "term_label": "plasma membrane",
  "gene": "UniProtKB:Q99767",
  "gene_name": "Amyloid-beta A4 precursor protein-binding family A member 2",
  "term_id": "GO:0005886"
}